cellular response to UV [GO:0034644] (biological process) Definition: Any process that results in a change in state or activity of a cell (in terms of movement, secretion, enzyme production, gene expression, etc.) as a result of an ultraviolet radiation (UV light) stimulus. Ultraviolet radiation is electromagnetic radiation with a wavelength in the range of 10 to 380 nanometers. Sources: GOC:mah Also known as: cellular response to UV light stimulus, cellular response to UV radiation stimulus, cellular response to ultraviolet light stimulus, cellular response to ultraviolet radiation stimulus Subtypes: GO:0007604, UV-damage excision repair [GO:0070914], cellular response to UV-A [GO:0071492], cellular response to UV-B [GO:0071493], cellular response to UV-C [GO:0071494] Relationships: is a type of response to UV [GO:0009411]; is a type of cellular response to light stimulus [GO:0071482]